positive regulation of flocculation [GO:1900735] (biological process) Also known as: up regulation of flocculation, up regulation of flocculation via cell wall protein-carbohydrate interaction, up-regulation of flocculation, up-regulation of flocculation via cell wall protein-carbohydrate interaction, upregulation of flocculation, upregulation of flocculation via cell wall protein-carbohydrate interaction, activation of flocculation, activation of flocculation via cell wall protein-carbohydrate interaction, positive regulation of flocculation via cell wall protein-carbohydrate interaction Relationships: is a type of positive regulation of cell-cell adhesion [GO:0022409]; is a type of regulation of flocculation [GO:0060256]; positively regulates flocculation [GO:0000128] Definition: Any process that activates or increases the frequency, rate or extent of flocculation. References: PMID:10591965, PMID:15466424, PMID:16568252 Sources: GOC:TermGenie, GOC:dgf